{
  "gene": "UniProtKB:Q9UBN6",
  "gene_name": "Tumor necrosis factor receptor superfamily member 10D",
  "term_id": "GO:0009986",
  "gene_symbol": "TNFRSF10D",
  "term_label": "cell surface"
}